{
  "gene_name": "Signal transducer and activator of transcription 4",
  "gene": "UniProtKB:Q14765",
  "gene_symbol": "STAT4",
  "term_id": "GO:0000978",
  "term_label": "RNA polymerase II cis-regulatory region sequence-specific DNA binding"
}